{
  "gene_name": "E3 ubiquitin-protein ligase MARCHF9",
  "term_label": "Golgi stack",
  "gene_symbol": "MARCHF9",
  "gene": "UniProtKB:Q86YJ5",
  "term_id": "GO:0005795"
}